L-cysteine catabolic process via cystine, using glutathione-cystine transhydrogenase [GO:0019454] (biological process) Definition: The chemical reactions and pathways resulting in the breakdown, via the compound cystine, of L-cysteine, catalyzed by the enzyme glutathione-cystine transhydrogenase. Relationships: is a type of GO:0019453; has part glutathione-cystine transhydrogenase activity [GO:0047141] Also known as: L-cysteine breakdown via cystine, using glutathione-cystine transhydrogenase, L-cysteine degradation via cystine, using glutathione-cystine transhydrogenase Sources: GOC:jl